{
  "term_id": "GO:0003883",
  "gene": "UniProtKB:P17812",
  "gene_symbol": "CTPS1",
  "term_label": "CTP synthase activity",
  "gene_name": "CTP synthase 1"
}